{
  "gene_name": "Olfactory receptor 7D4",
  "term_label": "olfactory receptor activity",
  "gene": "UniProtKB:Q8NG98",
  "term_id": "GO:0004984",
  "gene_symbol": "OR7D4"
}